{
  "gene_name": "GTP-binding protein SAR1b",
  "gene_symbol": "SAR1B",
  "gene": "UniProtKB:Q9Y6B6",
  "term_label": "endoplasmic reticulum to Golgi vesicle-mediated transport",
  "term_id": "GO:0006888"
}